mitotic cell cycle, embryonic [GO:0045448] (biological process) Subtypes: preblastoderm mitotic cell cycle [GO:0035185], GO:0035186 Regulation: regulated by regulation of mitotic cell cycle, embryonic [GO:0009794]; negatively regulated by negative regulation of mitotic cell cycle, embryonic [GO:0045976]; positively regulated by positive regulation of mitotic cell cycle, embryonic [GO:0045977] Sources: GOC:go_curators Definition: The eukaryotic cell cycle in which a cell is duplicated without changing ploidy, occurring in the embryo. Relationships: is a type of GO:0000278; is part of embryo development [GO:0009790]